kinetochore [GO:0000776] (cellular component) Relationships: is a type of intracellular membraneless organelle [GO:0043232]; is a type of supramolecular complex [GO:0099080]; is part of condensed chromosome, centromeric region [GO:0000779] Also known as: condensed chromosome kinetochore, condensed nuclear chromosome kinetochore, NMS complex Sources: GOC:elh Note: Note that the kinetochore overlaps the centromeric DNA, but centromeric DNA is not part of the kinetochore. Definition: A multisubunit complex that is located at the centromeric region of DNA and provides an attachment point for the spindle microtubules.